{
  "gene_name": "Ankyrin repeat domain-containing protein 34C",
  "gene": "UniProtKB:P0C6C1",
  "term_label": "Unknown biological process",
  "gene_symbol": "ANKRD34C",
  "term_id": "UNKNOWN:0002"
}